{
  "term_label": "transcription elongation factor activity",
  "gene_symbol": "EAF2",
  "term_id": "GO:0003711",
  "gene": "UniProtKB:Q96CJ1",
  "gene_name": "ELL-associated factor 2"
}